regulation of metanephros size [GO:0035566] (BP) Also known as: regulation of metanephric kidney size Definition: Any process that modulates the size of a metanephric kidney. Relationships: is a type of regulation of kidney size [GO:0035564]; is part of metanephros morphogenesis [GO:0003338] Sources: GOC:bf